aspartate-phenylpyruvate transaminase activity [GO:0047319] (molecular function) Also known as: aspartate:phenylpyruvate aminotransferase activity, L-aspartate:phenylpyruvate aminotransferase activity, aspartate--phenylpyruvate aminotransferase activity Relationships: is a type of transaminase activity [GO:0008483] Definition: Catalysis of the reaction: keto-phenylpyruvate + L-aspartate = L-phenylalanine + oxaloacetate. Sources: RHEA:14097